inorganic cation import across plasma membrane [GO:0098659] (biological process) Definition: The directed movement of inorganic cations from outside of a cell, across the plasma membrane and into the cytosol. Also known as: inorganic cation import into cell Relationships: is a type of inorganic ion import across plasma membrane [GO:0099587] Sources: GOC:dos Subtypes: zinc ion import across plasma membrane [GO:0071578], calcium ion import across plasma membrane [GO:0098703], copper ion import across plasma membrane [GO:0098705], iron ion import across plasma membrane [GO:0098711], GO:0098716, sodium ion import across plasma membrane [GO:0098719], ammonium import across plasma membrane [GO:0140157], manganese import into cell [GO:0140967], potassium ion import across plasma membrane [GO:1990573]